diacetyl reductase ((R)-acetoin forming) (NAD+) activity [GO:0052587] (molecular function) Sources: RHEA:22900 Also known as: (R)-acetoin dehydrogenase activity Definition: Catalysis of the reaction: (R)-acetoin + NAD+ = diacetyl + H+ + NADH. This reaction is catalyzed in the reverse direction. Relationships: is_a GO:0019152